{
  "term_id": "GO:0030527",
  "gene": "UniProtKB:P23527",
  "gene_name": "Histone H2B type 1-O",
  "term_label": "structural constituent of chromatin",
  "gene_symbol": "H2BC17"
}